{
  "term_label": "hydrolase activity",
  "gene_symbol": "ENPP5",
  "gene_name": "Ectonucleotide pyrophosphatase_phosphodiesterase family member 5",
  "gene": "UniProtKB:Q9UJA9",
  "term_id": "GO:0016787"
}